{
  "gene": "UniProtKB:Q9H115",
  "gene_symbol": "NAPB",
  "gene_name": "Beta-soluble NSF attachment protein",
  "term_id": "GO:0019905",
  "term_label": "syntaxin binding"
}